{
  "term_label": "negative regulation of small GTPase mediated signal transduction",
  "term_id": "GO:0051058",
  "gene_symbol": "ARHGAP45",
  "gene_name": "Rho GTPase-activating protein 45",
  "gene": "UniProtKB:Q92619"
}